{
  "term_label": "flavin adenine dinucleotide binding",
  "gene_name": "FAD-linked sulfhydryl oxidase ALR",
  "gene": "UniProtKB:P55789",
  "gene_symbol": "GFER",
  "term_id": "GO:0050660"
}